{
  "term_label": "mitochondrial inner membrane",
  "gene_symbol": "COX6B1",
  "gene_name": "Cytochrome c oxidase subunit 6B1",
  "term_id": "GO:0005743",
  "gene": "UniProtKB:P14854"
}